{
  "gene_name": "Organic cation_carnitine transporter 2",
  "term_id": "GO:0015651",
  "gene_symbol": "SLC22A5",
  "gene": "UniProtKB:O76082",
  "term_label": "quaternary ammonium group transmembrane transporter activity"
}